bis(monoacylglycero)phosphate synthase activity [GO:0160121] (molecular function) Relationships: is a type of acyltransferase activity, transferring groups other than amino-acyl groups [GO:0016747] Definition: Catalysis of the reaction: 2 3-acyl-sn-glycero-1-phospho-(1'-sn-glycerol) = 3-acyl-sn-glycero-1-phospho-(3'-acyl-1'-sn-glycerol) + sn-glycero-1-phospho-(1'-sn-glycerol). References: PMID:37708259 Sources: RHEA:77619